gamma-delta T cell lineage commitment [GO:0002365] (biological process) Definition: The process in which a pro-T cell becomes committed to becoming a gamma-delta T cell. Also known as: gamma-delta T lymphocyte lineage commitment, gamma-delta T-cell lineage commitment, gamma-delta T-lymphocyte lineage commitment Sources: GOC:add, ISBN:0781735149 Relationships: is_a T cell lineage commitment [GO:0002360]; is part of gamma-delta T cell differentiation [GO:0042492]